{
  "term_label": "cytoplasm",
  "gene_symbol": "FGF7",
  "gene": "UniProtKB:P21781",
  "term_id": "GO:0005737",
  "gene_name": "Fibroblast growth factor 7"
}